{
  "term_id": "GO:0016020",
  "gene_name": "Membrane-associated progesterone receptor component 2",
  "gene_symbol": "PGRMC2",
  "term_label": "membrane",
  "gene": "UniProtKB:O15173"
}